{
  "term_id": "GO:0005911",
  "gene": "UniProtKB:Q14168",
  "term_label": "cell-cell junction",
  "gene_symbol": "MPP2",
  "gene_name": "MAGUK p55 subfamily member 2"
}